{
  "term_id": "GO:0090200",
  "term_label": "positive regulation of release of cytochrome c from mitochondria",
  "gene_name": "Protein AF1q",
  "gene": "UniProtKB:Q13015",
  "gene_symbol": "MLLT11"
}